{
  "gene": "UniProtKB:Q8NC54",
  "gene_symbol": "KCT2",
  "gene_name": "Keratinocyte-associated transmembrane protein 2",
  "term_id": "UNKNOWN:0002",
  "term_label": "Unknown biological process"
}